{
  "gene": "UniProtKB:P42898",
  "gene_name": "Methylenetetrahydrofolate reductase (NADPH)",
  "gene_symbol": "MTHFR",
  "term_id": "GO:0071949",
  "term_label": "FAD binding"
}